positive regulation of deacetylase activity [GO:0090045] (BP) Relationships: is a type of positive regulation of catalytic activity [GO:0043085]; is a type of regulation of deacetylase activity [GO:0150065]; positively regulates deacetylase activity [GO:0019213] Sources: GOC:BHF, GOC:dph, GOC:tb Definition: Any process that activates or increases the frequency, rate or extent of deacetylase activity, the catalysis of the hydrolysis of an acetyl group or groups from a substrate molecule.